{
  "gene_name": "Serine_threonine-protein kinase 17B",
  "gene": "UniProtKB:O94768",
  "term_id": "GO:0005634",
  "gene_symbol": "STK17B",
  "term_label": "nucleus"
}